{
  "term_id": "GO:0000902",
  "term_label": "cell morphogenesis",
  "gene_symbol": "CAP1",
  "gene_name": "Adenylyl cyclase-associated protein 1",
  "gene": "UniProtKB:Q01518"
}